maltose import across plasma membrane [GO:0106081] (biological process) References: PMID:11136464 Definition: The directed movement of maltose from outside of a cell, across the plasma membrane and into the cytosol. Relationships: is a type of GO:0098704; is a type of GO:1904981